epithelial cell migration involved in mesonephric distal tubule morphogenesis [GO:0061279] (biological process) Definition: The orderly movement of epithelial cells within a renal tubule that contributes to mesonephric distal tubule morphogenesis. Sources: GOC:mtg_kidney_jan10 Relationships: is a type of epithelial cell migration involved in mesonephric nephron tubule morphogenesis [GO:0061278]; is_a epithelial cell migration involved in distal tubule morphogenesis [GO:0072157]; BFO_0000050 mesonephric distal tubule morphogenesis [GO:0061273]